{
  "gene_symbol": "UBE3B",
  "term_id": "GO:0061630",
  "term_label": "ubiquitin protein ligase activity",
  "gene_name": "Ubiquitin-protein ligase E3B",
  "gene": "UniProtKB:Q7Z3V4"
}